kainate selective glutamate receptor complex [GO:0032983] (cellular component) Definition: An assembly of four or five subunits which form a structure with an extracellular N-terminus and a large loop that together form the ligand binding domain. The C-terminus is intracellular. The ionotropic glutamate receptor complex itself acts as a ligand gated ion channel; on binding glutamate, charged ions pass through a channel in the center of the receptor complex. Kainate receptors are multimeric assemblies of GluK1-3 (also called GluR5-7), GluK4 (KA1) and GluK5 (KA2) subunits. References: PMID:18655795 Sources: GOC:bf Relationships: is a type of GO:0008328; is a type of potassium channel complex [GO:0034705]; is a type of sodium channel complex [GO:0034706]